{
  "gene_symbol": "PML",
  "gene": "UniProtKB:P29590",
  "term_id": "GO:0045087",
  "term_label": "innate immune response",
  "gene_name": "Protein PML"
}